regulation of microtubule nucleation [GO:0010968] (biological process) Definition: Any process that modulates the rate, frequency or extent of microtubule nucleation. Microtubule nucleation is the 'de novo' formation of a microtubule, in which tubulin heterodimers form metastable oligomeric aggregates, some of which go on to support formation of a complete microtubule. Microtubule nucleation usually occurs from a specific site within a cell. Subtypes: positive regulation of microtubule nucleation [GO:0090063], GO:1905833 Relationships: is a type of GO:0031113; regulates microtubule nucleation [GO:0007020] Sources: GOC:dph, GOC:tb